{
  "gene_symbol": "NOX1",
  "gene": "UniProtKB:Q9Y5S8",
  "term_label": "plasma membrane",
  "gene_name": "NADPH oxidase 1",
  "term_id": "GO:0005886"
}